{
  "gene": "UniProtKB:Q9BPZ3",
  "term_label": "cytoplasm",
  "gene_symbol": "PAIP2",
  "gene_name": "Polyadenylate-binding protein-interacting protein 2",
  "term_id": "GO:0005737"
}